regulation of cell-substrate adhesion [GO:0010810] (biological process) Subtypes: regulation of cell-matrix adhesion [GO:0001952], positive regulation of cell-substrate adhesion [GO:0010811], negative regulation of cell-substrate adhesion [GO:0010812], regulation of substrate adhesion-dependent cell spreading [GO:1900024], GO:1900187, regulation of substrate-dependent cell migration, cell attachment to substrate [GO:1904235] Definition: Any process that modulates the frequency, rate or extent of cell-substrate adhesion. Cell-substrate adhesion is the attachment of a cell to the underlying substrate via adhesion molecules. Relationships: is a type of regulation of cell adhesion [GO:0030155]; regulates cell-substrate adhesion [GO:0031589] Sources: GOC:dph, GOC:pf, GOC:tb